{
  "gene": "UniProtKB:Q969Z3",
  "term_label": "nitrate metabolic process",
  "gene_symbol": "MTARC2",
  "term_id": "GO:0042126",
  "gene_name": "Mitochondrial amidoxime reducing component 2"
}